{
  "term_id": "GO:0005615",
  "term_label": "extracellular space",
  "gene": "UniProtKB:P08697",
  "gene_symbol": "SERPINF2",
  "gene_name": "Alpha-2-antiplasmin"
}